2-oxoadipate dehydrogenase activity [GO:0160166] (molecular function) Relationships: is a type of oxidoreductase activity, acting on the aldehyde or oxo group of donors, disulfide as acceptor [GO:0016624] References: PMID:29191460, PMID:32695416 Sources: RHEA:69576 Definition: Catalysis of the reaction: 2-oxoadipate + H+ + N(6)-[(R)-lipoyl]-L-lysyl-[dihydrolipoyllysine-residue succinyltransferase] = CO2 + N(6)-[(R)-S(8)-glutaryldihydrolipoyl]-L-lysyl-[dihydrolipoyllysine-residue succinyltransferase].